interleukin-9 binding [GO:0019983] (molecular function) Relationships: is a type of GO:0019838; is a type of cytokine binding [GO:0019955] Also known as: IL-9 binding Definition: Binding to interleukin-9. Sources: GOC:jl